{
  "gene": "UniProtKB:P46926",
  "gene_symbol": "GNPDA1",
  "term_label": "N-acetylneuraminate catabolic process",
  "gene_name": "Glucosamine-6-phosphate isomerase 1",
  "term_id": "GO:0019262"
}